nuclear cyclin-dependent protein kinase holoenzyme complex [GO:0019908] (cellular component) Relationships: is a type of cyclin-dependent protein kinase holoenzyme complex [GO:0000307]; is a type of GO:0140513 Definition: Cyclin-dependent protein kinase (CDK) complex found in the nucleus. Sources: GOC:krc Subtypes: transcription factor TFIIH holo complex [GO:0005675], GO:0008024, CKM complex [GO:1990508] Also known as: CDK holoenzyme